{
  "term_id": "UNKNOWN:0003",
  "gene": "UniProtKB:Q13434",
  "term_label": "Unknown cellular component",
  "gene_name": "Putative E3 ubiquitin-protein ligase makorin-4",
  "gene_symbol": "MKRN4P"
}